{
  "term_id": "GO:0035371",
  "gene_name": "CDK5 regulatory subunit-associated protein 2",
  "gene_symbol": "CDK5RAP2",
  "gene": "UniProtKB:Q96SN8",
  "term_label": "microtubule plus-end"
}